{
  "term_label": "Unknown biological process",
  "gene_symbol": "EYS",
  "gene_name": "Protein eyes shut homolog",
  "gene": "UniProtKB:Q5T1H1",
  "term_id": "UNKNOWN:0002"
}